{
  "term_id": "UNKNOWN:0002",
  "term_label": "Unknown biological process",
  "gene_name": "LRRN4 C-terminal-like protein",
  "gene_symbol": "LRRN4CL",
  "gene": "UniProtKB:Q8ND94"
}